{
  "gene_name": "Uncharacterized protein",
  "gene_symbol": "A0A8V8TPW5",
  "gene": "UniProtKB:A0A8V8TPW5",
  "term_id": "UNKNOWN:0002",
  "term_label": "Unknown biological process"
}